5'-deoxyadenosine deaminase activity [GO:0090613] (molecular function) Relationships: is a type of hydrolase activity, acting on carbon-nitrogen (but not peptide) bonds, in cyclic amidines [GO:0016814]; is a type of deaminase activity [GO:0019239] Definition: Catalysis of the reaction: 5'deoxyadenosine + H2O = 5'deoxyinosine + NH3. References: PMID:23968233 Sources: RHEA:42892